{
  "gene": "UniProtKB:Q96HH9",
  "gene_symbol": "GRAMD2B",
  "gene_name": "GRAM domain-containing protein 2B",
  "term_label": "cytoplasmic microtubule",
  "term_id": "GO:0005881"
}